protein C inhibitor-KLK3 complex [GO:0036029] (cellular component) Also known as: PCI-KLK3 complex, SERPINA5-KLK3 complex, plasma serine protease inhibitor-KLK3 complex, protein C inhibitor-kallikrein-3 complex, protein C inhibitor-prostate-specific antigen complex, serpin A5-KLK3 complex References: PMID:1725227 Sources: GOC:ans Definition: A heterodimeric protein complex that contains protein C inhibitor (SERPINA5) and prostate-specific antigen (KLK3); formation of the complex inhibits the serine protease activity of prostate-specific antigen. Relationships: is a type of GO:0097180